{
  "gene": "UniProtKB:A8MQ03",
  "term_label": "Unknown cellular component",
  "gene_name": "Cysteine-rich tail protein 1",
  "gene_symbol": "CYSRT1",
  "term_id": "UNKNOWN:0003"
}